{
  "gene_symbol": "CSTF2",
  "term_id": "GO:0003729",
  "gene": "UniProtKB:P33240",
  "term_label": "mRNA binding",
  "gene_name": "Cleavage stimulation factor subunit 2"
}